GDP-mannose biosynthetic process from mannose [GO:0061728] (biological process) Definition: The chemical reactions and pathways resulting in the formation of GDP-mannose from mannose. References: PMID:16339137, PMID:24218558 Sources: GOC:dph Relationships: is a type of GO:0006013; is a type of GDP-mannose biosynthetic process [GO:0009298]; has part mannokinase activity [GO:0019158]